phosphotransferase activity, phosphate group as acceptor [GO:0016776] (molecular function) Subtypes: GO:0000827, inositol hexakisphosphate kinase activity [GO:0000828], diphosphoinositol pentakisphosphate kinase activity [GO:0000829], nucleoside diphosphate kinase activity [GO:0004550], phosphomevalonate kinase activity [GO:0004631], phosphomethylpyrimidine kinase activity [GO:0008972], polyphosphate kinase activity [GO:0008976], thiamine-phosphate kinase activity [GO:0009030], ribose 1,5-bisphosphate phosphokinase activity [GO:0033863], polyphosphate:AMP phosphotransferase activity [GO:0043751], nucleoside triphosphate adenylate kinase activity [GO:0046899], GO:0047335, 5-methyldeoxycytidine-5'-phosphate kinase activity [GO:0047336], dolichyl-diphosphate-polyphosphate phosphotransferase activity [GO:0047337], deoxynucleoside phosphate kinase activity, ATP as phosphate donor [GO:0047507], GO:0047887, nucleoside monophosphate kinase activity [GO:0050145], thiamine-diphosphate kinase activity [GO:0050331], isopentenyl phosphate kinase activity [GO:0102043], phytyl-P kinase activity [GO:0102763], deoxynucleoside phosphate kinase activity, dGTP as phosphate donor [GO:0106367], deoxynucleoside phosphate kinase activity, dTTP as phosphate donor [GO:0106368], GO:0106369, GO:0141090 Relationships: is_a transferase activity, transferring phosphorus-containing groups [GO:0016772] Sources: EC:2.7.4.- Definition: Catalysis of the transfer of a phosphorus-containing group from one compound (donor) to a phosphate group (acceptor).